{
  "gene_name": "Maturin",
  "term_id": "GO:0045654",
  "gene": "UniProtKB:Q8N3F0",
  "gene_symbol": "MTURN",
  "term_label": "positive regulation of megakaryocyte differentiation"
}